{
  "term_id": "GO:0006493",
  "gene_name": "N-acetylgalactosaminyltransferase 7",
  "gene": "UniProtKB:Q86SF2",
  "gene_symbol": "GALNT7",
  "term_label": "protein O-linked glycosylation"
}